{
  "term_label": "calcineurin complex",
  "gene_name": "Protein phosphatase 3 catalytic subunit alpha",
  "gene": "UniProtKB:Q08209",
  "term_id": "GO:0005955",
  "gene_symbol": "PPP3CA"
}